glossopharyngeal nerve development [GO:0021563] (biological process) Definition: Various sensory and motor branches of the glossopharyngeal nerve supply nerve connections to the pharynx and back of the tongue. The branchial motor component contains motor fibers that innervate muscles that elevate the pharynx and larynx, and the tympanic branch supplies parasympathetic fibers to the otic ganglion. Relationships: is a type of cranial nerve development [GO:0021545] Sources: GOC:cls, GOC:dgh, GOC:dph, GOC:jid, GO_REF:0000021 Also known as: cranial nerve 9 development, cranial nerve IX development, CN IX development